{
  "term_label": "cell adhesion mediated by integrin",
  "gene_symbol": "ITGB7",
  "gene": "UniProtKB:P26010",
  "gene_name": "Integrin beta-7",
  "term_id": "GO:0033627"
}